{
  "gene_symbol": "WDFY4",
  "term_label": "antigen processing and presentation",
  "gene": "UniProtKB:Q6ZS81",
  "term_id": "GO:0019882",
  "gene_name": "WD repeat- and FYVE domain-containing protein 4"
}